{
  "gene_symbol": "ELMOD1",
  "gene": "UniProtKB:Q8N336",
  "term_label": "synapse",
  "gene_name": "ELMO domain-containing protein 1",
  "term_id": "GO:0045202"
}